negative regulation of interleukin-21 production [GO:0032705] (biological process) Sources: GOC:mah Definition: Any process that stops, prevents, or reduces the frequency, rate, or extent of interleukin-21 production. Relationships: is a type of negative regulation of cytokine production [GO:0001818]; is a type of regulation of interleukin-21 production [GO:0032665]; negatively regulates interleukin-21 production [GO:0032625] Also known as: down regulation of interleukin-21 production, down-regulation of interleukin-21 production, downregulation of interleukin-21 production, negative regulation of interleukin-21 biosynthetic process